negative regulation of response to propan-1-ol [GO:1901446] (biological process) Relationships: is a type of negative regulation of response to alcohol [GO:1901420]; is_a regulation of response to propan-1-ol [GO:1901445]; negatively regulates GO:1901427 Definition: Any process that stops, prevents or reduces the frequency, rate or extent of response to propan-1-ol. Sources: GOC:TermGenie, GOC:mengo_curators Also known as: down regulation of response to propan-1-ol, down-regulation of response to propan-1-ol, downregulation of response to propan-1-ol, inhibition of response to propan-1-ol